{
  "gene_symbol": "FGL2",
  "term_label": "extracellular matrix",
  "term_id": "GO:0031012",
  "gene": "UniProtKB:Q14314",
  "gene_name": "Fibroleukin"
}